positive regulation of intermediate mesodermal cell fate determination [GO:0048397] (biological process) Sources: GOC:dgh Definition: Any process that activates or increases the frequency, rate or extent of intermediate mesoderm cell fate determination. Relationships: is a type of positive regulation of mesodermal cell fate determination [GO:0048336]; is a type of regulation of intermediate mesodermal cell fate determination [GO:0048395]; positively regulates intermediate mesodermal cell fate determination [GO:0048394] Also known as: up regulation of intermediate mesodermal cell fate determination, up-regulation of intermediate mesodermal cell fate determination, upregulation of intermediate mesodermal cell fate determination, activation of intermediate mesodermal cell fate determination, stimulation of intermediate mesodermal cell fate determination